{
  "gene_symbol": "LHX6",
  "term_id": "GO:0006357",
  "term_label": "regulation of transcription by RNA polymerase II",
  "gene": "UniProtKB:Q9UPM6",
  "gene_name": "LIM_homeobox protein Lhx6"
}